{
  "gene_symbol": "GNAO1",
  "term_id": "GO:0007212",
  "gene_name": "Guanine nucleotide-binding protein G(o) subunit alpha",
  "term_label": "G protein-coupled dopamine receptor signaling pathway",
  "gene": "UniProtKB:P09471"
}